{
  "gene_name": "Ubiquitin carboxyl-terminal hydrolase 19",
  "gene_symbol": "USP19",
  "term_id": "UNKNOWN:0003",
  "term_label": "Unknown cellular component",
  "gene": "UniProtKB:O94966"
}